{
  "gene_symbol": "SNX24",
  "term_id": "GO:1901981",
  "gene": "UniProtKB:Q9Y343",
  "term_label": "phosphatidylinositol phosphate binding",
  "gene_name": "Sorting nexin-24"
}